regulation of juvenile hormone secretion [GO:0007558] (biological process) Definition: Any process that modulates the frequency, rate or extent of juvenile hormone secretion. Relationships: is a type of regulation of lipid transport [GO:0032368]; is a type of regulation of endocrine process [GO:0044060]; is a type of regulation of hormone secretion [GO:0046883]; regulates GO:0045443 Subtypes: negative regulation of juvenile hormone secretion [GO:0045972], positive regulation of juvenile hormone secretion [GO:0045973] Sources: GOC:go_curators